L-aspartate:fumarate antiporter activity [GO:0062057] (MF) Relationships: is_a GO:0015138; is a type of L-aspartate transmembrane transporter activity [GO:0015183]; is a type of antiporter activity [GO:0015297] References: PMID:29995997 Definition: Enables the transport of L-aspartate and fumarate across a membrane according to the reaction L-aspartate (out) + fumarate (in) = L-aspartate (in) + fumarate (out).